{
  "gene_name": "Disintegrin and metalloproteinase domain-containing protein 18",
  "gene_symbol": "ADAM18",
  "term_id": "GO:0007155",
  "term_label": "cell adhesion",
  "gene": "UniProtKB:Q9Y3Q7"
}